lactic acid secretion [GO:0046722] (biological process) Definition: The controlled release of lactic acid, 2-hydroxypropanoic acid, by a cell or a tissue. Also known as: lactate secretion Sources: GOC:ai Relationships: is a type of GO:0035879; is a type of acid secretion [GO:0046717]